{
  "term_label": "actin filament organization",
  "gene_name": "Rho-related GTP-binding protein RhoG",
  "term_id": "GO:0007015",
  "gene": "UniProtKB:P84095",
  "gene_symbol": "RHOG"
}